{
  "term_id": "UNKNOWN:0001",
  "gene_symbol": "RBM17",
  "term_label": "Unknown molecular function",
  "gene": "UniProtKB:Q96I25",
  "gene_name": "Splicing factor 45"
}